lactosylceramide 1,3-N-acetyl-beta-D-glucosaminyltransferase activity [GO:0047256] (molecular function) Also known as: LA2 synthase activity, UDP-N-acetyl-D-glucosamine:D-galactosyl-1,4-beta-D-glucosylceramide beta-1,3-acetylglucosaminyltransferase activity, beta1->3-N-acetylglucosaminyltransferase activity, lactosylceramide beta-acetylglucosaminyltransferase activity, uridine diphosphoacetylglucosamine-lactosylceramide beta-acetylglucosaminyltransferase activity Relationships: is a type of acetylglucosaminyltransferase activity [GO:0008375] Sources: RHEA:13905 Definition: Catalysis of the reaction: a beta-D-Gal-(1->4)-beta-D-Glc-(1<->1)-Cer(d18:1(4E)) + UDP-N-acetyl-alpha-D-glucosamine = a beta-D-GlcNAc-(1->3)-beta-D-Gal-(1->4)-beta-D-Glc-(1<->1)-Cer(d18:1(4E)) + H+ + UDP.